{
  "gene_name": "HLA class II histocompatibility antigen, DQ alpha 1 chain",
  "gene": "UniProtKB:P01909",
  "gene_symbol": "HLA-DQA1",
  "term_label": "peptide antigen assembly with MHC class II protein complex",
  "term_id": "GO:0002503"
}